{
  "term_id": "GO:0000922",
  "term_label": "spindle pole",
  "gene_symbol": "CKAP5",
  "gene": "UniProtKB:Q14008",
  "gene_name": "Cytoskeleton-associated protein 5"
}